{
  "gene_name": "WD repeat-containing protein 70",
  "gene_symbol": "WDR70",
  "gene": "UniProtKB:Q9NW82",
  "term_id": "GO:0035861",
  "term_label": "site of double-strand break"
}